venom-mediated muscle damage in another organism [GO:0044521] (biological process) Subtypes: venom-mediated myocyte killing in another organism [GO:0044522] References: PMID:10620318, PMID:21150580 Sources: GOC:fj, GOC:jl Also known as: envenomation resulting in muscle damage in another organism, envenomation resulting in muscle damage in other organism Definition: A process that begins with venom being forced into an organism by the bite or sting of another organism, and ends with resultant muscle damage in the bitten organism. Relationships: is a type of venom-mediated disruption of anatomical structure in another organism [GO:0140138]